{
  "gene_symbol": "TERB2",
  "gene": "UniProtKB:Q8NHR7",
  "term_id": "UNKNOWN:0001",
  "gene_name": "Telomere repeats-binding bouquet formation protein 2",
  "term_label": "Unknown molecular function"
}